regulation of lung alveolus development [GO:1904653] (biological process) Relationships: is a type of GO:0050793; regulates lung alveolus development [GO:0048286] Subtypes: negative regulation of lung alveolus development [GO:1904654], GO:1904655 Definition: Any process that modulates the frequency, rate or extent of lung alveolus development. Also known as: regulation of alveolarization, regulation of alveologenesis References: PMID:23962064 Sources: GOC:TermGenie, GO_REF:0000058